{
  "gene_name": "Fibronectin type III and SPRY domain-containing protein 2",
  "term_id": "UNKNOWN:0003",
  "gene_symbol": "FSD2",
  "gene": "UniProtKB:A1L4K1",
  "term_label": "Unknown cellular component"
}